{
  "gene_symbol": "TLK1",
  "term_id": "GO:0004674",
  "gene_name": "Serine_threonine-protein kinase tousled-like 1",
  "term_label": "protein serine/threonine kinase activity",
  "gene": "UniProtKB:Q9UKI8"
}